{
  "term_label": "mitotic cell cycle",
  "gene_name": "Tubulin alpha chain-like 3",
  "gene_symbol": "TUBAL3",
  "term_id": "GO:0000278",
  "gene": "UniProtKB:A6NHL2"
}